{
  "gene_symbol": "ATG12",
  "term_id": "GO:0061723",
  "gene_name": "Ubiquitin-like protein ATG12",
  "term_label": "glycophagy",
  "gene": "UniProtKB:O94817"
}